{
  "term_label": "cytoskeleton",
  "gene": "UniProtKB:Q658L1",
  "gene_name": "Stabilizer of axonemal microtubules 2",
  "gene_symbol": "SAXO2",
  "term_id": "GO:0005856"
}